{
  "gene_symbol": "SLC1A2",
  "gene_name": "Excitatory amino acid transporter 2",
  "gene": "UniProtKB:P43004",
  "term_id": "GO:0005313",
  "term_label": "L-glutamate transmembrane transporter activity"
}